{
  "gene": "UniProtKB:Q9Y5F2",
  "gene_name": "Protocadherin beta-11",
  "term_id": "GO:0050839",
  "gene_symbol": "PCDHB11",
  "term_label": "cell adhesion molecule binding"
}